monooxygenase activity [GO:0004497] (molecular function) Definition: Catalysis of the incorporation of one atom of molecular oxygen (O2) into the substrate and the reduction of the other atom of O2 to water. References: PMID:1444267 Also known as: hydroxylase activity, mixed-function oxidase Relationships: is_a GO:0016491 Subtypes: GO:0004097, coumarin 7-hydroxylase activity [GO:0008389], GO:0008391, GO:0008395, retinoic acid 4-hydroxylase activity [GO:0008401], 3-demethoxyubiquinol 3-hydroxylase activity [GO:0008682], beta-carotene 3-hydroxylase activity [GO:0010291], GO:0016703, oxidoreductase activity, acting on paired donors, with incorporation or reduction of molecular oxygen, NAD(P)H as one donor, and incorporation of one atom of oxygen [GO:0016709], oxidoreductase activity, acting on paired donors, with incorporation or reduction of molecular oxygen, reduced flavin or flavoprotein as one donor, and incorporation of one atom of oxygen [GO:0016712], oxidoreductase activity, acting on paired donors, with incorporation or reduction of molecular oxygen, reduced iron-sulfur protein as one donor, and incorporation of one atom of oxygen [GO:0016713], oxidoreductase activity, acting on paired donors, with incorporation or reduction of molecular oxygen, reduced pteridine as one donor, and incorporation of one atom of oxygen [GO:0016714], GO:0016715, GO:0016716, ammonia monooxygenase activity [GO:0018597], 4-methoxybenzoate monooxygenase (O-demethylating) activity [GO:0018690], limonene monooxygenase activity [GO:0019113], deoxyhypusine monooxygenase activity [GO:0019135], ornithine N5-monooxygenase activity [GO:0031172], GO:0044875, luciferin monooxygenase activity [GO:0045289], p-coumarate 3-hydroxylase activity [GO:0046409], ferulate 5-hydroxylase activity [GO:0046424], phylloquinone monooxygenase (2,3-epoxidizing) activity [GO:0047097], 2-hydroxypyridine 5-monooxygenase activity [GO:0047546], 3-hydroxybenzoate 2-monooxygenase activity [GO:0047563], kynurenine 7,8-hydroxylase activity [GO:0050016], inositol oxygenase activity [GO:0050113], thiophene-2-carbonyl-CoA monooxygenase activity [GO:0050603], taxadiene 5-alpha-hydroxylase activity [GO:0050604], jasmonoyl-isoleucine-12-hydroxylase activity [GO:0052694], fatty acid in-chain hydroxylase activity [GO:0052722], all-trans retinoic acid 18-hydroxylase activity [GO:0062183], GO:0062185, linoleic acid epoxygenase activity [GO:0071614], 20-hydroxy-leukotriene B4 omega oxidase activity [GO:0097258], 20-aldehyde-leukotriene B4 20-monooxygenase activity [GO:0097259], acyl-lipid omega-(9-4) desaturase activity [GO:0102431], GO:0102733, eupatolide synthase activity [GO:0106244], GO:0140382